{
  "term_id": "GO:0000423",
  "gene_symbol": "ATG9B",
  "term_label": "mitophagy",
  "gene": "UniProtKB:Q674R7",
  "gene_name": "Autophagy-related protein 9B"
}